{
  "term_label": "Unknown molecular function",
  "term_id": "UNKNOWN:0001",
  "gene": "UniProtKB:Q6NXR4",
  "gene_name": "TELO2-interacting protein 2",
  "gene_symbol": "TTI2"
}